chloroplast thylakoid lumen [GO:0009543] (cellular component) Sources: GOC:mtg_sensu, ISBN:0943088399 Definition: The cavity enclosed within the chloroplast thylakoid membrane. An example of this component is found in Arabidopsis thaliana. Relationships: is a type of plastid thylakoid lumen [GO:0031978]; is part of chloroplast thylakoid [GO:0009534]